primary ovarian follicle growth involved in double layer follicle stage [GO:0043929] (biological process) Relationships: is a type of primary ovarian follicle growth [GO:0001545]; is part of double layer follicle stage [GO:0048161] Definition: Increase in size of primary follicles including oocyte growth and granulosa and/or theca cell proliferation until more than one layer of granulosa cells is present (preantral follicle), as part of the double layer follicle stage of oogenesis. Also known as: primary ovarian follicle growth during double layer follicle stage Sources: GOC:mtg_mpo